{
  "term_id": "GO:0010508",
  "gene": "UniProtKB:Q8NHG7",
  "gene_name": "Small VCP_p97-interacting protein",
  "gene_symbol": "SVIP",
  "term_label": "positive regulation of autophagy"
}